{
  "gene_symbol": "WDR25",
  "term_id": "UNKNOWN:0003",
  "gene": "UniProtKB:Q64LD2",
  "gene_name": "WD repeat-containing protein 25",
  "term_label": "Unknown cellular component"
}